{
  "gene_name": "Nectin-2",
  "term_label": "receptor ligand activity",
  "gene": "UniProtKB:Q92692",
  "term_id": "GO:0048018",
  "gene_symbol": "NECTIN2"
}